{
  "gene_name": "Zinc finger protein 891",
  "gene": "UniProtKB:A8MT65",
  "term_id": "GO:0006357",
  "gene_symbol": "ZNF891",
  "term_label": "regulation of transcription by RNA polymerase II"
}